attachment of meiotic spindle microtubules to kinetochore [GO:0051316] (biological process) Definition: The cellular process in which spindle microtubules become physically associated with the proteins making up the kinetochore complex in meiosis. Sources: GOC:ai, GOC:dph, GOC:tb Also known as: attachment of spindle microtubules to meiotic chromosome, attachment of spindle microtubules to kinetochore during meiosis, attachment of spindle microtubules to kinetochore during meiotic chromosome segregation Relationships: is_a attachment of spindle microtubules to kinetochore [GO:0008608]; is_a GO:1903046; is part of meiotic metaphase chromosome alignment [GO:0051311] Subtypes: spindle attachment to meiosis I kinetochore [GO:0051455], attachment of meiotic spindle microtubules to meiosis II kinetochore [GO:0051456]